{
  "gene_symbol": "KLHDC3",
  "term_id": "GO:0003682",
  "gene": "UniProtKB:Q9BQ90",
  "gene_name": "Kelch domain-containing protein 3",
  "term_label": "chromatin binding"
}